{
  "gene_symbol": "SAMD8",
  "gene_name": "Sphingomyelin synthase-related protein 1",
  "gene": "UniProtKB:Q96LT4",
  "term_id": "GO:0033188",
  "term_label": "sphingomyelin synthase activity"
}